{
  "gene": "UniProtKB:Q8NFU4",
  "term_id": "UNKNOWN:0002",
  "gene_name": "Follicular dendritic cell secreted peptide",
  "gene_symbol": "FDCSP",
  "term_label": "Unknown biological process"
}